{
  "term_label": "Unknown molecular function",
  "gene_name": "Pyridoxal-dependent decarboxylase domain-containing protein 1",
  "gene_symbol": "PDXDC1",
  "term_id": "UNKNOWN:0001",
  "gene": "UniProtKB:Q6P996"
}